{
  "gene_symbol": "LUZP4",
  "term_label": "Unknown cellular component",
  "gene_name": "Leucine zipper protein 4",
  "gene": "UniProtKB:Q9P127",
  "term_id": "UNKNOWN:0003"
}